hyoscyamine (6S)-dioxygenase activity [GO:0047998] (MF) Also known as: L-hyoscyamine,2-oxoglutarate:oxygen oxidoreductase ((6S)-hydroxylating), hyoscyamine (6S)-hydroxylase activity, hyoscyamine 6-beta-hydroxylase activity, hyoscyamine 6-hydroxylase activity, hyoscyamine 6beta-dioxygenase activity, hyoscyamine 6beta-hydroxylase activity Sources: EC:1.14.11.11, RHEA:12629 Relationships: is a type of 2-oxoglutarate-dependent dioxygenase activity [GO:0016706] Definition: Catalysis of the reaction: 2-oxoglutarate + L-hyoscyamine + O2 = (6S)-6-hydroxyhyoscyamine + CO2 + succinate.